{
  "gene": "UniProtKB:Q14008",
  "gene_name": "Cytoskeleton-associated protein 5",
  "term_label": "mitotic spindle organization",
  "gene_symbol": "CKAP5",
  "term_id": "GO:0007052"
}